D-galacturonate metabolic process [GO:0046396] (biological process) Relationships: is a type of GO:0005996; is a type of monocarboxylic acid metabolic process [GO:0032787] Subtypes: D-galacturonate catabolic process [GO:0019698], D-galacturonate biosynthetic process [GO:0033482] Sources: GOC:ai, GOC:jsg, GOC:mah, ISBN:0198506732 Also known as: D-galacturonate metabolism Definition: The chemical reactions and pathways involving D-galacturonate, the D-enantiomer of galacturonate, the anion of galacturonic acid. D-galacturonic acid is a component of plant gums and bacterial cell walls.